{
  "term_label": "positive regulation of cytosolic calcium ion concentration",
  "gene_name": "Atypical chemokine receptor 4",
  "gene_symbol": "ACKR4",
  "term_id": "GO:0007204",
  "gene": "UniProtKB:Q9NPB9"
}